{
  "gene_name": "SWI_SNF-related matrix-associated actin-dependent regulator of chromatin subfamily B member 1",
  "gene": "UniProtKB:Q12824",
  "gene_symbol": "SMARCB1",
  "term_id": "GO:0005634",
  "term_label": "nucleus"
}